regulation of granulocyte chemotaxis [GO:0071622] (biological process) Relationships: is a type of GO:0002688; regulates GO:0071621 Definition: Any process that modulates the rate, frequency or extent of granulocyte chemotaxis. Granulocyte chemotaxis is the movement of a granulocyte in response to an external stimulus. Subtypes: positive regulation of macrophage chemotaxis [GO:0010759], negative regulation of granulocyte chemotaxis [GO:0071623], positive regulation of granulocyte chemotaxis [GO:0071624], regulation of neutrophil chemotaxis [GO:0090022], regulation of eosinophil chemotaxis [GO:2000422] Sources: GOC:mah